leukotriene metabolic process [GO:0006691] (BP) Definition: The chemical reactions and pathways involving leukotriene, a pharmacologically active substance derived from a polyunsaturated fatty acid, such as arachidonic acid. Relationships: is a type of icosanoid metabolic process [GO:0006690] Sources: GOC:ma Also known as: leukotriene metabolism Subtypes: leukotriene biosynthetic process [GO:0019370], leukotriene catabolic process [GO:0036100], leukotriene B4 metabolic process [GO:0036102], leukotriene A4 metabolic process [GO:1901751]